{
  "term_label": "ephrin receptor signaling pathway",
  "gene_name": "Ephrin-A2",
  "gene": "UniProtKB:O43921",
  "term_id": "GO:0048013",
  "gene_symbol": "EFNA2"
}